{
  "term_label": "cytosolic large ribosomal subunit",
  "gene": "UniProtKB:P83881",
  "term_id": "GO:0022625",
  "gene_symbol": "RPL36A",
  "gene_name": "Large ribosomal subunit protein eL42"
}